{
  "gene_symbol": "BBS7",
  "term_label": "BBSome",
  "term_id": "GO:0034464",
  "gene_name": "Bardet-Biedl syndrome 7 protein",
  "gene": "UniProtKB:Q8IWZ6"
}